{
  "gene_name": "D site-binding protein",
  "gene": "UniProtKB:Q10586",
  "term_label": "DNA-binding transcription factor activity, RNA polymerase II-specific",
  "gene_symbol": "DBP",
  "term_id": "GO:0000981"
}